{
  "term_id": "UNKNOWN:0003",
  "gene_name": "Putative uncharacterized protein encoded by LINC00587",
  "gene_symbol": "LINC00587",
  "gene": "UniProtKB:B1AMM8",
  "term_label": "Unknown cellular component"
}